glycerol ether catabolic process [GO:0044269] (biological process) Definition: The chemical reactions and pathways resulting in the breakdown of glycerol ethers, any anhydride formed between two organic hydroxy compounds, one of which is glycerol. Sources: GOC:jl Also known as: glycerol ether breakdown, glycerol ether catabolism, glycerol ether degradation Relationships: is a type of ether catabolic process [GO:1901502] Subtypes: GO:0062234